beta-D-Gal-(1->4)-beta-D-GlcNAc-(1->3)-beta-D-Gal-(1->4)-D-Glc binding [GO:2001079] (molecular function) Definition: Binding to beta-D-Gal-(1->4)-beta-D-GlcNAc-(1->3)-beta-D-Gal-(1->4)-D-Glc. Relationships: is a type of GO:0097367 Sources: GOC:mengo_curators